{
  "term_label": "Unknown cellular component",
  "term_id": "UNKNOWN:0003",
  "gene_name": "Myotonin-protein kinase",
  "gene": "UniProtKB:Q09013",
  "gene_symbol": "DMPK"
}